cyclin-dependent protein serine/threonine kinase activity [GO:0004693] (molecular function) Definition: Cyclin-dependent catalysis of the reactions: ATP + protein serine = ADP + protein serine phosphate, and ATP + protein threonine = ADP + protein threonine phosphate. Relationships: is a type of protein serine/threonine kinase activity [GO:0004674]; is a type of cyclin-dependent protein kinase activity [GO:0097472] Note: This reaction requires the binding of a regulatory cyclin subunit and full activity requires stimulatory phosphorylation by a CDK-activating kinase (CAK). References: PMID:7877684, PMID:9841670 Sources: GOC:pr, GOC:rn Regulation: regulated by GO:0000079; negatively regulated by cyclin-dependent protein serine/threonine kinase inhibitor activity [GO:0004861]; regulated by GO:0016538; negatively regulated by negative regulation of cyclin-dependent protein serine/threonine kinase activity [GO:0045736]; positively regulated by positive regulation of cyclin-dependent protein serine/threonine kinase activity [GO:0045737]; positively regulated by cyclin-dependent protein serine/threonine kinase activator activity [GO:0061575] Also known as: cyclin-dependent kinase activity, cyclin-dependent protein kinase activity, CDK activity, CDK, catalytic subunit activity, cyclin-dependent protein kinase, intrinsic catalyst activity, D-type cyclin kinase activity, cdc2 kinase activity, cyclin D-cdk6 kinase activity, cyclin D-dependent kinase activity, cyclin E kinase activity, cyclin-A associated kinase activity, cyclin-dependent kinase 6 activity, cyclin-dependent kinase-2 activity, cyclin-dependent kinase-4 activity, neuronal cdc2-like kinase activity, ATP:cyclin phosphotransferase activity, CDK, Cdk-activating protein kinase activity, cdk-activating kinase activity